fructoselysine biosynthetic process [GO:1901282] (biological process) Sources: GOC:TermGenie, GOC:yaf, UniPathway:UPA00784 Relationships: is a type of fructosamine biosynthetic process [GO:0030391]; is a type of GO:0030393; is a type of carboxylic acid biosynthetic process [GO:0046394] Also known as: fructosyllysine anabolism, fructosyllysine biosynthesis, fructosyllysine biosynthetic process, fructosyllysine formation, fructosyllysine synthesis Definition: The chemical reactions and pathways resulting in the formation of fructoselysine.